{
  "gene": "UniProtKB:Q11203",
  "gene_symbol": "ST3GAL3",
  "term_label": "sialyltransferase activity",
  "term_id": "GO:0008373",
  "gene_name": "CMP-N-acetylneuraminate-beta-1,4-galactoside alpha-2,3-sialyltransferase"
}